{
  "gene_name": "Neurogenin-2",
  "term_id": "GO:0030900",
  "gene_symbol": "NEUROG2",
  "gene": "UniProtKB:Q9H2A3",
  "term_label": "forebrain development"
}